MAML3-RBP-Jkappa-ICN4 complex [GO:0071182] (cellular component) Relationships: is a type of nuclear protein-containing complex [GO:0140513] Also known as: MAML3-RBP-Jkappa-Notch4 complex Definition: A protein complex that consists of the intracellular domain of Notch4 (ICN4), the DNA-binding transcription factor RBP-Jkappa, and the transcriptional coactivator Mastermind-like-3 (MAML3); the complex is involved in transcriptional activation in response to Notch-mediated signaling. References: PMID:12370315